{
  "gene": "UniProtKB:Q9NVD7",
  "gene_symbol": "PARVA",
  "term_label": "substrate adhesion-dependent cell spreading",
  "gene_name": "Alpha-parvin",
  "term_id": "GO:0034446"
}